{
  "gene_symbol": "KLHL30-AS1",
  "term_label": "Unknown molecular function",
  "gene_name": "Putative uncharacterized protein KLHL30-AS1",
  "term_id": "UNKNOWN:0001",
  "gene": "UniProtKB:Q8NEE0"
}